{
  "term_label": "RNA binding",
  "gene_symbol": "RPS10P5",
  "gene": "UniProtKB:Q9NQ39",
  "term_id": "GO:0003723",
  "gene_name": "Putative ribosomal protein eS10-like"
}